{
  "gene_symbol": "DUSP14",
  "term_id": "UNKNOWN:0002",
  "term_label": "Unknown biological process",
  "gene_name": "Dual specificity protein phosphatase 14",
  "gene": "UniProtKB:O95147"
}